cellular response to vitamin D [GO:0071305] (biological process) Sources: GOC:mah Relationships: is a type of GO:0033280; is a type of cellular response to vitamin [GO:0071295]; is a type of cellular response to lipid [GO:0071396]; is a type of cellular response to oxygen-containing compound [GO:1901701] Definition: Any process that results in a change in state or activity of a cell (in terms of movement, secretion, enzyme production, gene expression, etc.) as a result of a vitamin D stimulus. Also known as: cellular response to calciferol, cellular response to cholecalciferol, cellular response to ergocalciferol